{
  "gene_symbol": "INPP5J",
  "term_id": "GO:0034485",
  "gene": "UniProtKB:Q15735",
  "term_label": "phosphatidylinositol-3,4,5-trisphosphate 5-phosphatase activity",
  "gene_name": "Phosphatidylinositol 4,5-bisphosphate 5-phosphatase A"
}